{
  "gene": "UniProtKB:P35398",
  "term_label": "nuclear receptor activity",
  "gene_symbol": "RORA",
  "gene_name": "Nuclear receptor ROR-alpha",
  "term_id": "GO:0004879"
}